{
  "term_id": "GO:0045944",
  "gene_symbol": "ASXL3",
  "gene": "UniProtKB:Q9C0F0",
  "term_label": "positive regulation of transcription by RNA polymerase II",
  "gene_name": "Putative Polycomb group protein ASXL3"
}